integrin alpha6-beta4 complex [GO:0034676] (cellular component) References: PMID:12297042 Also known as: alpha6-beta4 integrin complex, ITGA6-ITGB4 complex Relationships: is a type of integrin complex [GO:0008305] Definition: An integrin complex that comprises one alpha6 subunit and one beta4 subunit.